{
  "gene": "UniProtKB:Q9Y6H6",
  "term_id": "GO:0097623",
  "gene_symbol": "KCNE3",
  "term_label": "potassium ion export across plasma membrane",
  "gene_name": "Potassium voltage-gated channel subfamily E member 3"
}